{
  "gene_symbol": "MYO18A",
  "term_id": "GO:0016460",
  "gene_name": "Unconventional myosin-XVIIIa",
  "gene": "UniProtKB:Q92614",
  "term_label": "myosin II complex"
}